regulation of potassium:proton exchanging ATPase activity [GO:1904451] (biological process) References: PMID:11897793 Sources: GOC:TermGenie, GO_REF:0000059 Also known as: regulation of proton pump activity, regulation of (K+ + H+)-ATPase activity, regulation of ATP phosphohydrolase (H+/K+-exchanging), regulation of H+-K+-ATPase activity, regulation of H+/K(+)-ATPase activity, regulation of H+/K(+)-exchanging ATPase activity, regulation of H+/K+-ATPase activity, regulation of H+/K+-exchanging ATPase activity, regulation of H,K-ATPase activity, regulation of hydrogen/potassium-exchanging ATPase activity, regulation of hydrogen:potassium exchanging ATPase activity, regulation of hydrogen:potassium-exchanging ATPase activity, regulation of gastric H+/K(+) ATPase activity, regulation of gastric H+/K+ ATPase Definition: Any process that modulates the frequency, rate or extent of hydrogen:potassium-exchanging ATPase activity. Relationships: is a type of GO:0010155; is a type of regulation of transmembrane transporter activity [GO:0022898]; is a type of regulation of ATP-dependent activity [GO:0043462]; regulates P-type potassium:proton transporter activity [GO:0008900]